{
  "term_label": "cytosol",
  "gene": "UniProtKB:Q99541",
  "term_id": "GO:0005829",
  "gene_name": "Perilipin-2",
  "gene_symbol": "PLIN2"
}